alpha2-beta1 integrin-chondroadherin complex [GO:0071079] (cellular component) Definition: A protein complex that consists of an alpha2-beta1 integrin complex bound to the cartilage matrix protein chondroadherin. Relationships: is a type of plasma membrane protein complex [GO:0098797] References: PMID:9281592 Also known as: ITGA2-ITGB1-CHAD complex